candicidin catabolic process [GO:1901126] (biological process) Sources: GOC:TermGenie, GOC:yaf, UniPathway:UPA00101 Relationships: is a type of catabolic process [GO:0009056] Definition: The chemical reactions and pathways resulting in the breakdown of candicidin. Also known as: candicidin breakdown, candicidin catabolism, candicidin degradation